{
  "term_id": "GO:0016323",
  "gene_name": "Anion exchange protein 2",
  "term_label": "basolateral plasma membrane",
  "gene": "UniProtKB:P04920",
  "gene_symbol": "SLC4A2"
}